{
  "term_label": "Unknown biological process",
  "term_id": "UNKNOWN:0002",
  "gene_name": "Leucine-rich repeat-containing protein 25",
  "gene": "UniProtKB:Q8N386",
  "gene_symbol": "LRRC25"
}